{
  "gene": "UniProtKB:Q16739",
  "gene_name": "Ceramide glucosyltransferase",
  "gene_symbol": "UGCG",
  "term_id": "GO:0016020",
  "term_label": "membrane"
}